{
  "gene_symbol": "HTR3A",
  "gene_name": "5-hydroxytryptamine receptor 3A",
  "term_id": "GO:0005886",
  "gene": "UniProtKB:P46098",
  "term_label": "plasma membrane"
}